{
  "gene_symbol": "PSKH1",
  "gene": "UniProtKB:P11801",
  "term_label": "cytoplasm",
  "gene_name": "Serine_threonine-protein kinase H1",
  "term_id": "GO:0005737"
}